negative regulation of ERBB3 signaling pathway [GO:1905579] (biological process) Also known as: down regulation of ERBB3 signaling pathway, down regulation of ERBB3 signalling pathway, down regulation of HER3 signaling pathway, down regulation of receptor tyrosine-protein kinase erbB-3 signaling pathway, down-regulation of ERBB3 signaling pathway, down-regulation of ERBB3 signalling pathway, down-regulation of HER3 signaling pathway, down-regulation of receptor tyrosine-protein kinase erbB-3 signaling pathway, downregulation of ERBB3 signaling pathway, downregulation of ERBB3 signalling pathway, downregulation of HER3 signaling pathway, downregulation of receptor tyrosine-protein kinase erbB-3 signaling pathway, negative regulation of ERBB3 signalling pathway, negative regulation of HER3 signaling pathway, negative regulation of receptor tyrosine-protein kinase erbB-3 signaling pathway, inhibition of ERBB3 signaling pathway, inhibition of ERBB3 signalling pathway, inhibition of HER3 signaling pathway, inhibition of receptor tyrosine-protein kinase erbB-3 signaling pathway References: PMID:27353365 Sources: GOC:TermGenie, GOC:als, GO_REF:0000058 Definition: Any process that stops, prevents or reduces the frequency, rate or extent of ERBB3 signaling pathway. Relationships: is_a negative regulation of ERBB signaling pathway [GO:1901185]; is a type of regulation of ERBB3 signaling pathway [GO:1905578]; negatively regulates ERBB3 signaling pathway [GO:0038129]